{
  "term_id": "GO:0030953",
  "gene": "UniProtKB:O95359",
  "term_label": "astral microtubule organization",
  "gene_symbol": "TACC2",
  "gene_name": "Transforming acidic coiled-coil-containing protein 2"
}